{
  "term_label": "extracellular matrix",
  "term_id": "GO:0031012",
  "gene_symbol": "GPC1",
  "gene": "UniProtKB:P35052",
  "gene_name": "Glypican-1"
}